{
  "term_id": "GO:0000149",
  "gene": "UniProtKB:Q8N9I0",
  "term_label": "SNARE binding",
  "gene_name": "Synaptotagmin-2",
  "gene_symbol": "SYT2"
}